{
  "term_label": "Unknown biological process",
  "term_id": "UNKNOWN:0002",
  "gene_name": "N-acetylglucosamine-1-phosphotransferase subunit gamma",
  "gene_symbol": "GNPTG",
  "gene": "UniProtKB:Q9UJJ9"
}